{
  "gene": "UniProtKB:Q92623",
  "gene_name": "Tetratricopeptide repeat protein 9A",
  "term_label": "Unknown cellular component",
  "term_id": "UNKNOWN:0003",
  "gene_symbol": "TTC9"
}